long-chain fatty aldehyde dehydrogenase (NAD+) activity [GO:0050061] (molecular function) Relationships: is_a fatty aldehyde dehydrogenase (NAD+) activity [GO:0102673] Also known as: long-chain-aldehyde dehydrogenase activity, fatty aldehyde:NAD+ oxidoreductase activity, long-chain aliphatic aldehyde dehydrogenase activity, long-chain fatty aldehyde dehydrogenase activity, long-chain-aldehyde:NAD+ oxidoreductase activity Sources: RHEA:10652 Definition: Catalysis of the reaction: a long-chain fatty aldehyde + H2O + NAD+ = a long-chain fatty acid + 2 H+ + NADH. Subtypes: GO:0047104